HCN channel complex [GO:0098855] (cellular component) References: PMID:20829353 Relationships: is a type of voltage-gated potassium channel complex [GO:0008076] Definition: A cation ion channel with a preference for K+ over Na+ ions, which is activated by membrane hyperpolarization, and consists of a tetramer of HCN family members. Some members of this family (HCN1, HCN2 and HCN4) are also activated when cAMP binds to their cyclic nucleotide binding domain (CNBD). Channel complexes of this family play an important role in the control of pacemaker activity in the heart. Also known as: K/Na hyperpolarization-activated cyclic nucleotide-gated channel complex, potassium/sodium hyperpolarization-activated cyclic nucleotide-gated channel complex, HCN1 channel complex, HCN2 channel complex, HCN3 channel complex, HCN4 channel complex, K/Na hyperpolarization-activated channel 3 complex, K/Na hyperpolarization-activated cyclic nucleotide-gated channel 1 complex, K/Na hyperpolarization-activated cyclic nucleotide-gated channel 2 complex, K/Na hyperpolarization-activated cyclic nucleotide-gated channel 4 complex, potassium/sodium hyperpolarization-activated channel 3 complex, potassium/sodium hyperpolarization-activated cyclic nucleotide-gated channel 1 complex, potassium/sodium hyperpolarization-activated cyclic nucleotide-gated channel 2 complex, potassium/sodium hyperpolarization-activated cyclic nucleotide-gated channel 4 complex, potassium/sodium hyperpolarization-activated cyclic nucleotide-gated channel 2 tetramer, potassium/sodium hyperpolarization-activated cyclic nucleotide-gated channel 4 tetramer